{
  "term_id": "GO:0005741",
  "gene_symbol": "CYB5B",
  "gene": "UniProtKB:O43169",
  "term_label": "mitochondrial outer membrane",
  "gene_name": "Cytochrome b5 type B"
}